{
  "term_label": "Unknown molecular function",
  "gene_name": "Golgi-associated RAB2 interactor protein 5B",
  "gene": "UniProtKB:Q8N5Q1",
  "gene_symbol": "GARIN5B",
  "term_id": "UNKNOWN:0001"
}